regulation of systemic arterial blood pressure by atrial natriuretic peptide [GO:0003050] (biological process) Sources: GOC:mtg_cardio Also known as: blood pressure regulation by atrial natriuretic peptide, blood pressure regulation by ANP Relationships: is a type of regulation of systemic arterial blood pressure by hormone [GO:0001990] Definition: The regulation of blood pressure mediated by the signaling molecule atrial natriuretic peptide.